{
  "gene_symbol": "KCNK7",
  "term_label": "outward rectifier potassium channel activity",
  "term_id": "GO:0015271",
  "gene_name": "Potassium channel subfamily K member 7",
  "gene": "UniProtKB:Q9Y2U2"
}